{
  "gene_name": "Tumor necrosis factor alpha-induced protein 8",
  "term_label": "cytoplasm",
  "gene_symbol": "TNFAIP8",
  "term_id": "GO:0005737",
  "gene": "UniProtKB:O95379"
}